{
  "term_label": "DNA-binding transcription repressor activity, RNA polymerase II-specific",
  "gene_name": "Zinc finger protein 589",
  "gene_symbol": "ZNF589",
  "term_id": "GO:0001227",
  "gene": "UniProtKB:Q86UQ0"
}